mannonate dehydratase activity [GO:0008927] (molecular function) Relationships: is_a hydro-lyase activity [GO:0016836] Definition: Catalysis of the reaction: D-mannonate = 2-dehydro-3-deoxy-D-gluconate + H2O. Also known as: D-mannonate hydro-lyase (2-dehydro-3-deoxy-D-gluconate-forming), D-mannonate hydro-lyase activity, D-mannonate hydrolyase activity, altronate hydrolase activity, altronic hydro-lyase activity, mannonate hydrolyase activity, mannonic hydrolase activity Sources: EC:4.2.1.8, RHEA:20097